{
  "gene_symbol": "PPIAL4A",
  "gene": "UniProtKB:Q9Y536",
  "term_id": "GO:0003755",
  "term_label": "peptidyl-prolyl cis-trans isomerase activity",
  "gene_name": "Peptidyl-prolyl cis-trans isomerase A-like 4A"
}